{
  "gene_symbol": "CORIN",
  "term_id": "GO:0005886",
  "gene": "UniProtKB:Q9Y5Q5",
  "gene_name": "Atrial natriuretic peptide-converting enzyme",
  "term_label": "plasma membrane"
}